{
  "term_label": "Unknown biological process",
  "gene_name": "Phosphatidylglycerophosphatase and protein-tyrosine phosphatase 1",
  "term_id": "UNKNOWN:0002",
  "gene": "UniProtKB:Q8WUK0",
  "gene_symbol": "PTPMT1"
}